{
  "term_id": "UNKNOWN:0002",
  "gene_name": "T cell receptor beta joining 2-4",
  "gene_symbol": "TRBJ2-4",
  "gene": "UniProtKB:A0A0A0MT87",
  "term_label": "Unknown biological process"
}